{
  "gene": "UniProtKB:Q00G26",
  "gene_symbol": "PLIN5",
  "gene_name": "Perilipin-5",
  "term_id": "GO:0010890",
  "term_label": "positive regulation of triglyceride storage"
}